selenocysteine lyase activity [GO:0009000] (molecular function) Also known as: L-selenocysteine selenide-lyase (L-alanine-forming), selenocysteine beta-lyase activity, selenocysteine reductase activity Definition: Catalysis of the reaction: L-selenocysteine + reduced acceptor = hydrogen selenide + L-alanine + acceptor. Sources: EC:4.4.1.16 Relationships: is a type of GO:0016846